{
  "gene_symbol": "ZNF544",
  "term_label": "nucleus",
  "term_id": "GO:0005634",
  "gene": "UniProtKB:Q6NX49",
  "gene_name": "Zinc finger protein 544"
}